{
  "gene_name": "Prickle-like protein 4",
  "term_id": "GO:0030036",
  "gene": "UniProtKB:Q2TBC4",
  "gene_symbol": "PRICKLE4",
  "term_label": "actin cytoskeleton organization"
}